{
  "gene": "UniProtKB:O14793",
  "term_label": "skeletal muscle tissue development",
  "term_id": "GO:0007519",
  "gene_name": "Growth_differentiation factor 8",
  "gene_symbol": "MSTN"
}